farnesylcysteine lyase activity [GO:0102149] (molecular function) Definition: Catalysis of the reaction: S-[(2E,6E)-farnesyl]-L-cysteine + O2 + H2O = (2-trans,6-trans)-farnesal + L-cysteine + hydrogen peroxide. Sources: EC:1.8.3.6, GOC:pz Relationships: is a type of oxidoreductase activity, acting on a sulfur group of donors, oxygen as acceptor [GO:0016670]